{
  "term_id": "UNKNOWN:0002",
  "gene_name": "Putative uncharacterized protein BAALC-AS2",
  "term_label": "Unknown biological process",
  "gene": "UniProtKB:P0C853",
  "gene_symbol": "BAALC-AS2"
}